{
  "gene": "UniProtKB:P01705",
  "gene_symbol": "IGLV2-23",
  "term_label": "Unknown molecular function",
  "gene_name": "Immunoglobulin lambda variable 2-23",
  "term_id": "UNKNOWN:0001"
}